sarcosine biosynthetic process [GO:1901054] (BP) Definition: The chemical reactions and pathways resulting in the formation of sarcosine. Relationships: is a type of GO:0042398; is a type of non-proteinogenic amino acid biosynthetic process [GO:0170043]; is a type of sarcosine metabolic process [GO:1901052]; is a type of alpha-amino acid biosynthetic process [GO:1901607] References: PMID:31402327 Sources: GOC:TermGenie, GOC:yaf Also known as: sarcosine anabolism, sarcosine biosynthesis, sarcosine formation, sarcosine synthesis